{
  "term_label": "Unknown molecular function",
  "gene_symbol": "LINC00587",
  "gene": "UniProtKB:B1AMM8",
  "gene_name": "Putative uncharacterized protein encoded by LINC00587",
  "term_id": "UNKNOWN:0001"
}